{
  "term_label": "protein maturation",
  "gene_name": "Mitochondrial intermembrane space import and assembly protein 40",
  "gene": "UniProtKB:Q8N4Q1",
  "gene_symbol": "CHCHD4",
  "term_id": "GO:0051604"
}